monocarboxylic acid metabolic process [GO:0032787] (biological process) Sources: GOC:vk Subtypes: acetate metabolic process [GO:0006083], lactate metabolic process [GO:0006089], pyruvate metabolic process [GO:0006090], creatine metabolic process [GO:0006600], fatty acid metabolic process [GO:0006631], GO:0006768, bile acid metabolic process [GO:0008206], GO:0009441, gamma-aminobutyric acid metabolic process [GO:0009448], abscisic acid metabolic process [GO:0009687], salicylic acid metabolic process [GO:0009696], cinnamic acid metabolic process [GO:0009803], pantothenate metabolic process [GO:0015939], formate metabolic process [GO:0015942], benzoate metabolic process [GO:0018874], GO:0018887, 3-chloroacrylic acid metabolic process [GO:0018888], 2,4-dichlorophenoxyacetic acid metabolic process [GO:0018901], GO:0018924, L-tryptophan catabolic process to indole-3-acetate [GO:0019440], D-gluconate metabolic process [GO:0019521], L-histidine catabolic process to hydantoin-5-propionate [GO:0019560], glucuronate metabolic process [GO:0019585], shikimate metabolic process [GO:0019632], GO:0019636, unsaturated monocarboxylic acid metabolic process [GO:0032789], ferulate metabolic process [GO:0033494], kynurenic acid metabolic process [GO:0034275], penicillin metabolic process [GO:0042316], retinoic acid metabolic process [GO:0042573], anthranilate metabolic process [GO:0043420], GO:0046278, D-galacturonate metabolic process [GO:0046396], para-aminobenzoic acid metabolic process [GO:0046482], glyoxylate metabolic process [GO:0046487], F420-0 metabolic process [GO:0052645], monocarboxylic acid catabolic process [GO:0072329], GO:0072330, indolebutyric acid metabolic process [GO:0080024], 4-hydroxyphenylacetate metabolic process [GO:1901022], GO:1901847 Relationships: is a type of carboxylic acid metabolic process [GO:0019752] Also known as: monocarboxylate metabolic process, monocarboxylic acid metabolism Definition: The chemical reactions and pathways involving monocarboxylic acids, any organic acid containing one carboxyl (COOH) group or anion (COO-).